{
  "gene_symbol": "VEZT",
  "term_label": "cell-cell adhesion",
  "gene_name": "Vezatin",
  "term_id": "GO:0098609",
  "gene": "UniProtKB:Q9HBM0"
}